{
  "gene": "UniProtKB:Q9BZD7",
  "gene_name": "Transmembrane gamma-carboxyglutamic acid protein 3",
  "term_label": "serine-type endopeptidase activity",
  "gene_symbol": "PRRG3",
  "term_id": "GO:0004252"
}